{
  "gene_name": "Separin",
  "gene": "UniProtKB:Q14674",
  "term_label": "mitotic spindle",
  "term_id": "GO:0072686",
  "gene_symbol": "ESPL1"
}